adiponectin secretion [GO:0070162] (biological process) Sources: GOC:BHF, GOC:rl Relationships: is a type of protein secretion [GO:0009306]; is a type of endocrine hormone secretion [GO:0060986] Regulation: regulated by regulation of adiponectin secretion [GO:0070163]; RO_0002212 by negative regulation of adiponectin secretion [GO:0070164]; positively regulated by GO:0070165 Definition: The regulated release of adiponectin, a protein hormone, by adipose tissue.